{
  "term_id": "GO:0140375",
  "gene_name": "Uncharacterized protein",
  "gene": "UniProtKB:A0A0G2JMM0",
  "gene_symbol": "LOC128966728",
  "term_label": "immune receptor activity"
}